alpha7-beta1 integrin-focal adhesion kinase complex [GO:0071135] (cellular component) Relationships: is a type of plasma membrane protein complex [GO:0098797] Also known as: ITGA7-ITGB1-PTK2 complex References: PMID:17598176 Definition: A protein complex that consists of an alpha7-beta1 integrin complex bound to focal adhesion kinase.